purine ribonucleoside metabolic process [GO:0046128] (biological process) Also known as: purine ribonucleoside metabolism Sources: GOC:ai Relationships: is a type of ribonucleoside metabolic process [GO:0009119]; is a type of purine nucleoside metabolic process [GO:0042278] Definition: The chemical reactions and pathways involving any ribonucleoside, a nucleoside in which purine base is linked to a ribose (beta-D-ribofuranose) molecule. Subtypes: guanosine metabolic process [GO:0008617], 7-methylguanosine metabolic process [GO:0008618], adenosine metabolic process [GO:0046085], inosine metabolic process [GO:0046102], purine ribonucleoside biosynthetic process [GO:0046129], purine ribonucleoside catabolic process [GO:0046130], S-adenosylhomocysteine metabolic process [GO:0046498], S-adenosylmethioninamine metabolic process [GO:0046499], 1-methylguanosine metabolic process [GO:0080179], 2-methylguanosine metabolic process [GO:0080180]